{
  "gene_symbol": "H2BC9",
  "gene_name": "Histone H2B type 1-H",
  "gene": "UniProtKB:Q93079",
  "term_id": "GO:0003677",
  "term_label": "DNA binding"
}